{
  "gene_name": "Zinc-regulated GTPase metalloprotein activator 1E",
  "gene_symbol": "ZNG1E",
  "term_label": "protein maturation",
  "gene": "UniProtKB:Q5RIA9",
  "term_id": "GO:0051604"
}